antigen processing and presentation of endogenous peptide antigen via MHC class Ib via ER pathway, TAP-dependent [GO:0002489] (biological process) Definition: The process in which an antigen-presenting cell expresses a peptide antigen of endogenous origin on its cell surface in association with an MHC class Ib protein complex following intracellular transport via a TAP (transporter associated with antigen processing) pathway. The peptide is typically a fragment of a larger endogenous protein which has been degraded within the cell and is dependent on TAP transport from the cytosol to ER for association with the MHC class Ib molecule. Class Ib here refers to non-classical class I molecules, such as those of the HLA-E gene family. Also known as: TAP-dependent antigen processing and presentation of endogenous peptide antigen via MHC class Ib via ER pathway, TAP-dependent endogenous peptide antigen processing and presentation via MHC class Ib via ER pathway, endogenous peptide antigen processing and presentation via MHC class Ib via ER pathway, TAP-dependent References: PMID:15928678 Sources: GOC:add Relationships: is_a GO:0002488